{
  "gene_symbol": "IFIH1",
  "gene_name": "Interferon-induced helicase C domain-containing protein 1",
  "gene": "UniProtKB:Q9BYX4",
  "term_label": "antiviral innate immune response",
  "term_id": "GO:0140374"
}